{
  "term_id": "GO:0071222",
  "term_label": "cellular response to lipopolysaccharide",
  "gene": "UniProtKB:Q04206",
  "gene_symbol": "RELA",
  "gene_name": "Transcription factor p65"
}